response to endogenous stimulus [GO:0009719] (BP) Subtypes: response to hormone [GO:0009725], GO:0055094, response to growth factor [GO:0070848], cellular response to endogenous stimulus [GO:0071495] Definition: Any process that results in a change in state or activity of a cell or an organism (in terms of movement, secretion, enzyme production, gene expression, etc.) as a result of a stimulus arising within the organism. Relationships: is a type of response to stimulus [GO:0050896] Note: Note that this term is in the subset of terms that should not be used for direct gene product annotation. Instead, select a child term or, if no appropriate child term exists, please request a new term. Direct annotations to this term may be amended during annotation QC. Sources: GOC:sm